{
  "gene_symbol": "HHIP",
  "gene": "UniProtKB:Q96QV1",
  "gene_name": "Hedgehog-interacting protein",
  "term_label": "Unknown cellular component",
  "term_id": "UNKNOWN:0003"
}